{
  "term_label": "cell differentiation",
  "gene_name": "Homeobox protein Nkx-2.2",
  "term_id": "GO:0030154",
  "gene": "UniProtKB:O95096",
  "gene_symbol": "NKX2-2"
}